anterior lateral line neuromast hair cell morphogenesis [GO:0035679] (biological process) Definition: The change in form (cell shape and size) that occurs when an anterior lateral line neuromast hair cell progresses from its initial formation to its mature state. A neuromast hair cell is a hair cell that acts as a sensory receptor of the neuromast; it is morphologically polarized as a result of the relative position of the single kinocilium and the clusters of stereocilia on its apical surface. Relationships: is a type of neuromast hair cell morphogenesis [GO:0035678]; is part of GO:0035676 Sources: ISBN:0125296509, ISBN:0387968377